{
  "gene_symbol": "CSRP1",
  "gene_name": "Cysteine and glycine-rich protein 1",
  "term_id": "GO:0008307",
  "gene": "UniProtKB:P21291",
  "term_label": "structural constituent of muscle"
}